{
  "term_id": "UNKNOWN:0003",
  "gene_symbol": "GLOD4",
  "term_label": "Unknown cellular component",
  "gene_name": "Glyoxalase domain-containing protein 4",
  "gene": "UniProtKB:Q9HC38"
}